ubiquitin activating enzyme binding [GO:0033134] (molecular function) Definition: Binding to a ubiquitin activating enzyme, any of the E1 proteins. Sources: GOC:mah Relationships: is a type of small protein activating enzyme binding [GO:0044388]